{
  "term_id": "GO:0006364",
  "gene": "UniProtKB:O95707",
  "gene_name": "Ribonuclease P protein subunit p29",
  "gene_symbol": "POP4",
  "term_label": "rRNA processing"
}